{
  "gene_name": "Keratin, type I cytoskeletal 10",
  "gene": "UniProtKB:P13645",
  "gene_symbol": "KRT10",
  "term_id": "GO:0030216",
  "term_label": "keratinocyte differentiation"
}